{
  "term_id": "GO:2000300",
  "gene": "UniProtKB:O00445",
  "gene_name": "Synaptotagmin-5",
  "term_label": "regulation of synaptic vesicle exocytosis",
  "gene_symbol": "SYT5"
}